axoneme [GO:0005930] (cellular component) Note: Note that cilia and eukaryotic flagella are deemed to be equivalent. In diplomonad species, such as Giardia, the axoneme may extend intracellularly up to 5um away from the plane of the plasma membrane. Definition: The bundle of microtubules and associated proteins that forms the core of cilia (also called flagella) in eukaryotic cells and is responsible for their movements. Sources: GOC:bf, GOC:cilia, ISBN:0198547684 Also known as: ciliary axoneme, cilium axoneme, flagellar axoneme, flagellum axoneme Relationships: is a type of cellular anatomical structure [GO:0110165]; is part of cytoskeleton [GO:0005856]; is part of ciliary plasm [GO:0097014]; has part microtubule [GO:0005874]